behavioral response to pain [GO:0048266] (biological process) Definition: Any process that results in a change in the behavior of an organism as a result of a pain stimulus. Pain stimuli cause activation of nociceptors, peripheral receptors for pain, include receptors which are sensitive to painful mechanical stimuli, extreme heat or cold, and chemical stimuli. Relationships: is a type of behavior [GO:0007610]; BFO_0000050 response to pain [GO:0048265] Subtypes: behavioral response to chemical pain [GO:0061366] Sources: GOC:jid Also known as: behavioural response to pain